{
  "term_label": "acetylcholine receptor signaling pathway",
  "gene_symbol": "LY6G6E",
  "gene": "UniProtKB:A0A0B4J1T7",
  "gene_name": "Lymphocyte antigen 6 family member G6E",
  "term_id": "GO:0095500"
}